positive regulation of CD4-positive, alpha-beta T cell costimulation [GO:1900281] (biological process) Also known as: positive regulation of CD4-positive, alpha beta T cell costimulation, up regulation of CD4-positive, alpha beta T cell costimulation, up-regulation of CD4-positive, alpha beta T cell costimulation, upregulation of CD4-positive, alpha beta T cell costimulation, activation of CD4-positive, alpha beta T cell costimulation Sources: GOC:BHF, GOC:TermGenie, GOC:pr Relationships: is a type of regulation of CD4-positive, alpha-beta T cell costimulation [GO:1900279]; is a type of GO:2000516; is a type of GO:2000525; positively regulates CD4-positive, alpha-beta T cell costimulation [GO:0035783] Definition: Any process that activates or increases the frequency, rate or extent of CD4-positive, alpha-beta T cell costimulation.